{
  "term_label": "acylglycerol homeostasis",
  "gene_name": "Apolipoprotein A-I",
  "term_id": "GO:0055090",
  "gene_symbol": "APOA1",
  "gene": "UniProtKB:P02647"
}